{
  "gene": "UniProtKB:Q96GS6",
  "gene_name": "Alpha_beta hydrolase domain-containing protein 17A",
  "term_id": "GO:0005886",
  "gene_symbol": "ABHD17A",
  "term_label": "plasma membrane"
}